{
  "term_label": "apical plasma membrane",
  "term_id": "GO:0016324",
  "gene_symbol": "RAPGEF2",
  "gene": "UniProtKB:Q9Y4G8",
  "gene_name": "Rap guanine nucleotide exchange factor 2"
}